{
  "term_label": "Unknown biological process",
  "term_id": "UNKNOWN:0002",
  "gene_symbol": "MBD4",
  "gene": "UniProtKB:O95243",
  "gene_name": "Methyl-CpG-binding domain protein 4"
}